{
  "gene_symbol": "SNU13",
  "term_label": "maturation of SSU-rRNA",
  "term_id": "GO:0030490",
  "gene": "UniProtKB:P55769",
  "gene_name": "NHP2-like protein 1"
}